{
  "term_id": "GO:0004674",
  "gene": "UniProtKB:Q09013",
  "term_label": "protein serine/threonine kinase activity",
  "gene_symbol": "DMPK",
  "gene_name": "Myotonin-protein kinase"
}